{
  "term_label": "mRNA cleavage and polyadenylation specificity factor complex",
  "term_id": "GO:0005847",
  "gene_name": "Cleavage and polyadenylation specificity factor subunit 1",
  "gene": "UniProtKB:Q10570",
  "gene_symbol": "CPSF1"
}